{
  "gene_name": "T cell receptor gamma joining P (Fragment)",
  "gene": "UniProtKB:A0A0C4DH63",
  "term_label": "Unknown molecular function",
  "term_id": "UNKNOWN:0001",
  "gene_symbol": "TRGJP"
}